hepatic stellate cell proliferation [GO:1990922] (biological process) Definition: The multiplication or reproduction of hepatic stellate cells, resulting in the expansion of a hepatic stellate cell population. Hepatic stellate cells are found in the perisinusoidal space of the liver, and are capable of multiple roles including storage of retinol, presentation of antigen to T cells (including CD1d-restricted NKT cells), and upon activation, production of extracellular matrix components. This cell type comprises approximately 8-15% of total cells in the liver. References: PMID:15358192, PMID:18466260 Sources: GOC:sl Also known as: Ito cell proliferation, hepatic perisinusoidal cell proliferation, perisinusoidal cell proliferation Relationships: is a type of fibroblast proliferation [GO:0048144] Regulation: regulated by regulation of hepatic stellate cell proliferation [GO:1904897]; negatively regulated by negative regulation of hepatic stellate cell proliferation [GO:1904898]; RO_0002213 by GO:1904899